{
  "gene_name": "Cation channel sperm-associated protein 1",
  "gene_symbol": "CATSPER1",
  "term_label": "regulation of cilium beat frequency involved in ciliary motility",
  "gene": "UniProtKB:Q8NEC5",
  "term_id": "GO:0060296"
}